{
  "gene_name": "Transmembrane protein 154",
  "gene_symbol": "TMEM154",
  "term_label": "Unknown biological process",
  "gene": "UniProtKB:Q6P9G4",
  "term_id": "UNKNOWN:0002"
}